{
  "term_id": "GO:0001725",
  "term_label": "stress fiber",
  "gene": "UniProtKB:O14639",
  "gene_symbol": "ABLIM1",
  "gene_name": "Actin-binding LIM protein 1"
}